{
  "term_id": "UNKNOWN:0003",
  "gene_symbol": "SCG5",
  "gene_name": "Neuroendocrine protein 7B2",
  "gene": "UniProtKB:P05408",
  "term_label": "Unknown cellular component"
}